{
  "term_id": "GO:0006357",
  "term_label": "regulation of transcription by RNA polymerase II",
  "gene": "UniProtKB:P17481",
  "gene_name": "Homeobox protein Hox-B8",
  "gene_symbol": "HOXB8"
}